negative regulation of border follicle cell delamination [GO:0030712] (biological process) Definition: Any process that decreases the frequency, rate or extent of border cell delamination. Relationships: is a type of positive regulation of cell-cell adhesion [GO:0022409]; is_a regulation of border follicle cell delamination [GO:0030710]; is a type of negative regulation of biological process [GO:0048519]; negatively regulates border follicle cell delamination [GO:0030709] References: PMID:10822261 Also known as: negative regulation of border cell delamination, down regulation of border follicle cell delamination, down-regulation of border follicle cell delamination, downregulation of border follicle cell delamination, inhibition of border follicle cell delamination